Notch signaling involved in heart development [GO:0061314] (biological process) Relationships: is a type of Notch signaling pathway [GO:0007219]; is a type of cell surface receptor signaling pathway involved in heart development [GO:0061311] Also known as: Notch signalling involved in heart development Definition: The series of molecular signals initiated by binding of an extracellular ligand to a Notch receptor on the surface of the target cell and contributing to the progression of the heart over time. Sources: GOC:mtg_heart Subtypes: Notch signaling pathway involved in regulation of secondary heart field cardioblast proliferation [GO:0003270]